{
  "gene_name": "Chorionic somatomammotropin hormone 1",
  "term_id": "GO:0046427",
  "term_label": "positive regulation of receptor signaling pathway via JAK-STAT",
  "gene_symbol": "CSH1",
  "gene": "UniProtKB:P0DML2"
}